{
  "gene_name": "Calsyntenin-2",
  "gene_symbol": "CLSTN2",
  "gene": "UniProtKB:Q9H4D0",
  "term_label": "positive regulation of synapse assembly",
  "term_id": "GO:0051965"
}